{
  "term_id": "GO:0002767",
  "gene_name": "Immunoglobulin subtype domain-containing protein",
  "gene_symbol": "A0A2R8YCY7",
  "gene": "UniProtKB:A0A2R8YCY7",
  "term_label": "immune response-inhibiting cell surface receptor signaling pathway"
}